{
  "gene_symbol": "HNRNPA1L3",
  "term_id": "GO:0000398",
  "gene": "UniProtKB:A0A2R8Y4L2",
  "term_label": "mRNA splicing, via spliceosome",
  "gene_name": "Heterogeneous nuclear ribonucleoprotein A1-like 3"
}